{
  "term_id": "GO:0008511",
  "gene_name": "Solute carrier family 12 member 3",
  "term_label": "sodium:potassium:chloride symporter activity",
  "gene_symbol": "SLC12A3",
  "gene": "UniProtKB:P55017"
}